{
  "term_label": "cell motility",
  "gene": "UniProtKB:Q9BYX7",
  "term_id": "GO:0048870",
  "gene_name": "Putative beta-actin-like protein 3",
  "gene_symbol": "POTEKP"
}